tRNA-dihydrouridine20b synthase activity [GO:0102267] (molecular function) Relationships: is a type of GO:0017150 Definition: Catalysis of the reaction: a 5,6-dihydrouracil20b in tRNA + NAD(P) = H+ + a uracil20b in tRNA + NAD(P)H. Sources: GOC:pz